{
  "term_id": "GO:0035725",
  "gene_name": "Amiloride-sensitive sodium channel subunit alpha",
  "gene_symbol": "SCNN1A",
  "gene": "UniProtKB:P37088",
  "term_label": "sodium ion transmembrane transport"
}